{
  "gene_name": "CMRF35-like molecule 7",
  "term_label": "plasma membrane",
  "term_id": "GO:0005886",
  "gene_symbol": "CD300LB",
  "gene": "UniProtKB:A8K4G0"
}